{
  "gene_name": "Inhibitor of growth protein 1",
  "gene": "UniProtKB:Q9UK53",
  "gene_symbol": "ING1",
  "term_id": "GO:0045893",
  "term_label": "positive regulation of DNA-templated transcription"
}